negative regulation of convergent extension involved in gastrulation [GO:1904104] (biological process) Definition: Any process that stops, prevents or reduces the frequency, rate or extent of convergent extension involved in gastrulation. Relationships: is_a regulation of convergent extension involved in gastrulation [GO:1904103]; is a type of negative regulation of morphogenesis of an epithelium [GO:1905331]; negatively regulates convergent extension involved in gastrulation [GO:0060027] Also known as: down regulation of convergent extension involved in gastrulation, down-regulation of convergent extension involved in gastrulation, downregulation of convergent extension involved in gastrulation, inhibition of convergent extension involved in gastrulation References: PMID:24892953 Sources: GOC:TermGenie, GOC:dph, GO_REF:0000058 Subtypes: negative regulation of convergent extension involved in somitogenesis [GO:1904128], negative regulation of convergent extension involved in neural plate elongation [GO:1904131], negative regulation of convergent extension involved in rhombomere morphogenesis [GO:1904134], negative regulation of convergent extension involved in notochord morphogenesis [GO:1904137]